{
  "gene_symbol": "ERP29",
  "term_id": "GO:0005783",
  "term_label": "endoplasmic reticulum",
  "gene": "UniProtKB:P30040",
  "gene_name": "Endoplasmic reticulum resident protein 29"
}